positive regulation of cell proliferation by VEGF-activated platelet derived growth factor receptor signaling pathway [GO:0038091] (biological process) Definition: The series of molecular signals initiated by vascular endothelial growth factor (VEGF) binding to a platelet-derived growth factor receptor (PDGFR) on the surface of a cell, which activates or increases the frequency, rate or extent of cell proliferation. References: PMID:17470632 Sources: GOC:signaling Also known as: positive regulation of cell proliferation by VEGF-activated platelet derived growth factor receptor signalling pathway, positive regulation of cell proliferation by VEGF/PDGFR signaling pathway, VEGF-A-induced cell proliferation Relationships: is a type of positive regulation of cell population proliferation [GO:0008284]; is a type of VEGF-activated platelet-derived growth factor receptor signaling pathway [GO:0038086]